{
  "gene_symbol": "CBLL1",
  "gene": "UniProtKB:Q75N03",
  "term_id": "GO:0030155",
  "gene_name": "E3 ubiquitin-protein ligase Hakai",
  "term_label": "regulation of cell adhesion"
}